{
  "gene": "UniProtKB:Q13427",
  "gene_symbol": "PPIG",
  "term_label": "protein folding",
  "term_id": "GO:0006457",
  "gene_name": "Peptidyl-prolyl cis-trans isomerase G"
}